{
  "gene_name": "Taurine up-regulated 1 protein",
  "term_label": "Unknown biological process",
  "term_id": "UNKNOWN:0002",
  "gene_symbol": "TUG1",
  "gene": "UniProtKB:A0A6I8PU40"
}